forebrain astrocyte fate commitment [GO:0021878] (biological process) References: PMID:16226447 Sources: GOC:cls, GOC:dgh, GOC:dph, GOC:jid, GO_REF:0000021 Relationships: is a type of GO:0060018; is part of GO:0021896 Definition: The process in which the developmental fate of a cell becomes restricted such that it will develop into an astrocyte that resides in the forebrain.